cyanocobalamin reductase (cyanide-eliminating) (NADP+) activity [GO:0033787] (molecular function) Sources: RHEA:16113 Also known as: NADPH2:cyanocob(III)alamin oxidoreductase (cyanide-eliminating) activity, NADPH:cyanocob(III)alamin oxidoreductase (cyanide-eliminating) activity, cob(I)alamin, cyanide:NADP+ oxidoreductase activity, cyanocobalamin reductase (NADPH, cyanide-eliminating) activity, cyanocobalamin reductase (NADPH; CN-eliminating) activity, cyanocobalamin reductase activity Relationships: is a type of oxidoreductase activity, acting on metal ions, NAD or NADP as acceptor [GO:0016723] Definition: Catalysis of the reaction: cob(I)alamin + hydrogen cyanide + NADP+ = cyanocob(III)alamin + H+ + NADPH.